{
  "term_id": "GO:0050911",
  "gene": "UniProtKB:Q8NH08",
  "gene_name": "Olfactory receptor 10AC1",
  "gene_symbol": "OR10AC1",
  "term_label": "detection of chemical stimulus involved in sensory perception of smell"
}